{
  "gene_name": "Neuroplastin",
  "gene": "UniProtKB:Q9Y639",
  "gene_symbol": "NPTN",
  "term_id": "GO:0007156",
  "term_label": "homophilic cell-cell adhesion"
}